{
  "term_label": "Unknown molecular function",
  "term_id": "UNKNOWN:0001",
  "gene_symbol": "NIN",
  "gene_name": "Ninein",
  "gene": "UniProtKB:Q8N4C6"
}